regulation of cell fate determination [GO:1905933] (biological process) Subtypes: regulation of mesodermal cell fate determination [GO:0048334], regulation of asymmetric protein localization involved in cell fate determination [GO:1904785], GO:1905934, positive regulation of cell fate determination [GO:1905935] Definition: Any process that modulates the frequency, rate or extent of cell fate determination. References: PMID:25793578 Sources: GOC:TermGenie, GOC:bhm, GO_REF:0000058 Relationships: is a type of GO:0050793; is a type of regulation of cellular process [GO:0050794]; regulates GO:0001709